{
  "term_label": "DNA-binding transcription factor activity, RNA polymerase II-specific",
  "term_id": "GO:0000981",
  "gene_name": "Tumor protein 63",
  "gene": "UniProtKB:Q9H3D4",
  "gene_symbol": "TP63"
}